{
  "term_id": "GO:0005634",
  "gene": "UniProtKB:P62807",
  "gene_symbol": "H2BC10",
  "gene_name": "Histone H2B type 1-C_E_F_G_I",
  "term_label": "nucleus"
}